T cell activation [GO:0042110] (biological process) Regulation: regulated by regulation of T cell activation [GO:0050863]; negatively regulated by negative regulation of T cell activation [GO:0050868]; positively regulated by positive regulation of T cell activation [GO:0050870] Subtypes: T cell activation involved in immune response [GO:0002286], T cell differentiation [GO:0030217], memory T cell activation [GO:0035709], T cell proliferation [GO:0042098], gamma-delta T cell activation [GO:0046629], alpha-beta T cell activation [GO:0046631] Relationships: is a type of GO:0046649 Definition: The change in morphology and behavior of a mature or immature T cell resulting from exposure to a mitogen, cytokine, chemokine, cellular ligand, or an antigen for which it is specific. Sources: GOC:mgi_curators, ISBN:0781735149 Also known as: T lymphocyte activation, T-cell activation, T-lymphocyte activation